aminoimidazolase activity [GO:0047664] (molecular function) Also known as: 4-aminoimidazole aminohydrolase activity, 4-aminoimidazole hydrolase activity Sources: RHEA:22348 Relationships: is a type of hydrolase activity, acting on carbon-nitrogen (but not peptide) bonds, in cyclic amidines [GO:0016814] Definition: Catalysis of the reaction:4-aminoimidazole + H20 = imidazol-4-one + NH3.